regulation of proline transport [GO:0070881] (biological process) Definition: Any process that modulates the frequency, rate or extent of proline transport. Relationships: is_a regulation of organic acid transport [GO:0032890]; is a type of GO:0051955; regulates GO:0015824 Sources: GOC:mah Subtypes: regulation of L-proline import across plasma membrane [GO:1905735]